{
  "gene_symbol": "ZFP36L2",
  "term_label": "nuclear-transcribed mRNA poly(A) tail shortening",
  "gene_name": "mRNA decay activator protein ZFP36L2",
  "term_id": "GO:0000289",
  "gene": "UniProtKB:P47974"
}